{
  "gene_name": "5-hydroxytryptamine receptor 1E",
  "term_id": "GO:0007268",
  "gene": "UniProtKB:P28566",
  "gene_symbol": "HTR1E",
  "term_label": "chemical synaptic transmission"
}